{
  "gene_symbol": "NSA2",
  "term_label": "preribosome, large subunit precursor",
  "term_id": "GO:0030687",
  "gene": "UniProtKB:O95478",
  "gene_name": "Ribosome biogenesis protein NSA2 homolog"
}